{
  "gene_symbol": "P3H3",
  "term_id": "GO:0019797",
  "term_label": "procollagen-proline 3-dioxygenase activity",
  "gene": "UniProtKB:Q8IVL6",
  "gene_name": "Prolyl 3-hydroxylase 3"
}